regulation of ventricular cardiac muscle cell membrane depolarization [GO:0060373] (biological process) Relationships: is a type of regulation of membrane depolarization [GO:0003254] Sources: GOC:dph, GOC:tb Also known as: regulation of ventricular cardiomyocyte membrane depolarization, electrocardiogram QRS complex, ventricular depolarization Definition: Any process that modulates the establishment or extent of a membrane potential in the depolarizing direction away from the resting potential in a ventricular cardiomyocyte.